positive regulation of thyroid gland epithelial cell proliferation [GO:1904443] (biological process) Relationships: is a type of positive regulation of epithelial cell proliferation [GO:0050679]; is a type of positive regulation of developmental process [GO:0051094]; is a type of GO:0051240; is a type of regulation of thyroid gland epithelial cell proliferation [GO:1904441]; positively regulates thyroid gland epithelial cell proliferation [GO:1990789] Definition: Any process that activates or increases the frequency, rate or extent of thyroid gland epithelial cell proliferation. Also known as: up regulation of thyroid gland epithelial cell proliferation, up-regulation of thyroid gland epithelial cell proliferation, upregulation of thyroid gland epithelial cell proliferation, activation of Hurthle cell proliferation, activation of thyroid follicular cell proliferation, activation of thyroid gland epithelial cell proliferation, positive regulation of Hurthle cell proliferation, positive regulation of thyroid follicular cell proliferation, up regulation of Hurthle cell proliferation, up regulation of thyroid follicular cell proliferation, up-regulation of Hurthle cell proliferation, up-regulation of thyroid follicular cell proliferation, upregulation of Hurthle cell proliferation, upregulation of thyroid follicular cell proliferation References: PMID:17646383 Sources: GOC:TermGenie, GO_REF:0000058